{
  "term_label": "ESC/E(Z) complex",
  "gene": "UniProtKB:Q16576",
  "term_id": "GO:0035098",
  "gene_symbol": "RBBP7",
  "gene_name": "Histone-binding protein RBBP7"
}